{
  "gene": "UniProtKB:Q96MN5",
  "gene_name": "Transcription elongation factor A N-terminal and central domain-containing protein 2",
  "term_id": "GO:0005634",
  "gene_symbol": "TCEANC2",
  "term_label": "nucleus"
}